{
  "gene_symbol": "ZBTB38",
  "term_id": "UNKNOWN:0003",
  "gene_name": "Zinc finger and BTB domain-containing protein 38",
  "gene": "UniProtKB:Q8NAP3",
  "term_label": "Unknown cellular component"
}